enterobactin synthetase complex [GO:0009366] (cellular component) Relationships: is a type of intracellular protein-containing complex [GO:0140535]; is a type of catalytic complex [GO:1902494] Definition: A multienzyme complex usually composed of four proteins, EntB, EntD, EntE and EntF. Plays a role in the enterobactin biosynthesis pathway. Also known as: enterochelin synthetase complex References: PMID:9485415